{
  "gene_symbol": "SIRT5",
  "gene_name": "NAD-dependent protein deacylase sirtuin-5, mitochondrial",
  "gene": "UniProtKB:Q9NXA8",
  "term_id": "GO:0017136",
  "term_label": "histone deacetylase activity, NAD-dependent"
}